{
  "term_id": "UNKNOWN:0002",
  "gene_symbol": "MYH9",
  "gene": "UniProtKB:P35579",
  "term_label": "Unknown biological process",
  "gene_name": "Myosin-9"
}